{
  "gene": "UniProtKB:Q7Z3Z4",
  "gene_symbol": "PIWIL4",
  "term_label": "regulatory ncRNA-mediated gene silencing",
  "gene_name": "Piwi-like protein 4",
  "term_id": "GO:0031047"
}